regulation of immune effector process [GO:0002697] (biological process) Subtypes: GO:0002631, negative regulation of immune effector process [GO:0002698], positive regulation of immune effector process [GO:0002699], GO:0002700, regulation of leukocyte mediated immunity [GO:0002703], GO:0030449, regulation of natural killer cell proliferation involved in immune response [GO:0032820], regulation of natural killer cell differentiation involved in immune response [GO:0032826], regulation of CD4-positive, CD25-positive, alpha-beta regulatory T cell differentiation involved in immune response [GO:0032832], regulation of leukocyte degranulation [GO:0043300], regulation of memory T cell differentiation [GO:0043380], regulation of T-helper cell differentiation [GO:0045622], GO:0060264, regulation of immune complex clearance by monocytes and macrophages [GO:0090264], regulation of melanotic encapsulation of foreign target [GO:0140539], GO:1900098, GO:1903027, regulation of Fc-gamma receptor signaling pathway involved in phagocytosis [GO:1905449], GO:2001188, regulation of gamma-delta T cell activation involved in immune response [GO:2001191] Definition: Any process that modulates the frequency, rate, or extent of an immune effector process. Sources: GOC:add Relationships: is a type of regulation of immune system process [GO:0002682]; regulates GO:0002252